{
  "term_label": "regulation of mRNA processing",
  "term_id": "GO:0050684",
  "gene_symbol": "SRPK2",
  "gene_name": "SRSF protein kinase 2",
  "gene": "UniProtKB:P78362"
}